{
  "gene_symbol": "PRKAA1",
  "term_label": "nucleotide-activated protein kinase complex",
  "gene_name": "5'-AMP-activated protein kinase catalytic subunit alpha-1",
  "term_id": "GO:0031588",
  "gene": "UniProtKB:Q13131"
}